{
  "gene_name": "Double-stranded RNA-specific adenosine deaminase",
  "term_label": "double-stranded RNA adenosine deaminase activity",
  "gene_symbol": "ADAR",
  "gene": "UniProtKB:P55265",
  "term_id": "GO:0003726"
}